2-aminoethylphosphonate transport [GO:0033223] (biological process) Definition: The directed movement of 2-aminoethylphosphonate, into, out of or within a cell, or between cells, by means of some agent such as a transporter or pore. Sources: GOC:mlg Also known as: 2-phosphonoethylamine transport, ciliatine transport Relationships: is a type of nitrogen compound transport [GO:0071705]